{
  "gene_name": "Granzyme K",
  "term_label": "serine-type endopeptidase activity",
  "term_id": "GO:0004252",
  "gene": "UniProtKB:P49863",
  "gene_symbol": "GZMK"
}